{
  "term_id": "GO:0005737",
  "gene": "UniProtKB:Q5T0D9",
  "gene_symbol": "TPRG1L",
  "gene_name": "Tumor protein p63-regulated gene 1-like protein",
  "term_label": "cytoplasm"
}